{
  "gene_name": "Zinc finger protein 670",
  "gene": "UniProtKB:Q9BS34",
  "term_id": "GO:0000981",
  "gene_symbol": "ZNF670",
  "term_label": "DNA-binding transcription factor activity, RNA polymerase II-specific"
}